{
  "term_id": "UNKNOWN:0002",
  "gene_name": "Heparan sulfate glucosamine 3-O-sulfotransferase 3B1",
  "gene": "UniProtKB:Q9Y662",
  "gene_symbol": "HS3ST3B1",
  "term_label": "Unknown biological process"
}